{
  "term_label": "AP-1 adaptor complex",
  "gene_name": "AP-3 complex subunit mu-2",
  "gene_symbol": "AP3M2",
  "term_id": "GO:0030121",
  "gene": "UniProtKB:P53677"
}